{
  "term_id": "UNKNOWN:0001",
  "gene_symbol": "MRFAP1",
  "gene": "UniProtKB:Q9Y605",
  "term_label": "Unknown molecular function",
  "gene_name": "MORF4 family-associated protein 1"
}